{
  "gene_name": "Putative N-acetyltransferase 8B",
  "term_label": "Unknown biological process",
  "gene": "UniProtKB:Q9UHF3",
  "term_id": "UNKNOWN:0002",
  "gene_symbol": "NAT8B"
}